{
  "gene_name": "Leukemia inhibitory factor",
  "term_label": "cytokine activity",
  "gene_symbol": "LIF",
  "term_id": "GO:0005125",
  "gene": "UniProtKB:P15018"
}